{
  "gene_symbol": "OR14J1",
  "gene_name": "Olfactory receptor 14J1",
  "term_id": "UNKNOWN:0003",
  "gene": "UniProtKB:Q9UGF5",
  "term_label": "Unknown cellular component"
}